{
  "gene": "UniProtKB:Q92544",
  "term_id": "UNKNOWN:0001",
  "gene_symbol": "TM9SF4",
  "term_label": "Unknown molecular function",
  "gene_name": "Transmembrane 9 superfamily member 4"
}